{
  "term_id": "UNKNOWN:0002",
  "gene_symbol": "SPATA17",
  "gene": "UniProtKB:Q96L03",
  "gene_name": "Spermatogenesis-associated protein 17",
  "term_label": "Unknown biological process"
}